chloroplast envelope [GO:0009941] (cellular component) Relationships: is a type of plastid envelope [GO:0009526]; is part of chloroplast [GO:0009507] Definition: The double lipid bilayer enclosing the chloroplast and separating its contents from the rest of the cytoplasm; includes the intermembrane space. Sources: GOC:tb